{
  "gene_name": "Inactive phospholipase C-like protein 1",
  "term_id": "GO:0004435",
  "gene_symbol": "PLCL1",
  "gene": "UniProtKB:Q15111",
  "term_label": "phosphatidylinositol-4,5-bisphosphate phospholipase C activity"
}